{
  "term_id": "GO:0003700",
  "gene": "UniProtKB:Q13422",
  "term_label": "DNA-binding transcription factor activity",
  "gene_name": "DNA-binding protein Ikaros",
  "gene_symbol": "IKZF1"
}